{
  "term_id": "GO:0006888",
  "gene": "UniProtKB:Q9H0V9",
  "term_label": "endoplasmic reticulum to Golgi vesicle-mediated transport",
  "gene_symbol": "LMAN2L",
  "gene_name": "VIP36-like protein"
}